{
  "gene": "UniProtKB:O60678",
  "gene_name": "Protein arginine N-methyltransferase 3",
  "gene_symbol": "PRMT3",
  "term_id": "GO:0006355",
  "term_label": "regulation of DNA-templated transcription"
}